{
  "term_label": "glucokinase activity",
  "gene": "UniProtKB:P52789",
  "gene_symbol": "HK2",
  "term_id": "GO:0004340",
  "gene_name": "Hexokinase-2"
}